symbiont-mediated suppression of host cAMP/PKA signal transduction [GO:0075210] (biological process) Also known as: disruption of host cAMP-mediated signal transduction, negative regulation by symbiont of host cAMP-mediated signal transduction, negative regulation by symbiont of host cAMP-mediated signaling, suppression by symbiont of host cAMP-mediated signal transduction, symbiont-mediated suppression of host PKA signal transduction, symbiont-mediated suppression of host cAMP signal transduction Relationships: is a type of symbiont-mediated suppression of host signal transduction pathway [GO:0052029] Note: Note that this term is used to annotate gene products of the symbiont. To annotate host gene products, consider the biological process term "Negative regulation by host of symbiont cAMP-mediated signal transduction ; GO:0075207". Definition: A process in which a symbiont interferes with, inhibits or disrupts a cAMP/PKA signal transduction in the host organism. The host is defined as the larger of the organisms involved in a symbiotic interaction. Sources: GOC:pamgo_curators